regulation of multicellular organism growth [GO:0040014] (biological process) Sources: GOC:dph, GOC:ems, GOC:tb Relationships: is a type of regulation of developmental growth [GO:0048638]; is_a GO:0051239; regulates multicellular organism growth [GO:0035264] Subtypes: GO:0040015, positive regulation of multicellular organism growth [GO:0040018] Also known as: regulation of body growth, regulation of body size Definition: Any process that modulates the frequency, rate or extent of growth of the body of an organism so that it reaches its usual body size.